{
  "term_id": "GO:0043197",
  "term_label": "dendritic spine",
  "gene_name": "Oligophrenin-1",
  "gene_symbol": "OPHN1",
  "gene": "UniProtKB:O60890"
}